negative regulation of tolerance induction to nonself antigen [GO:0002656] (biological process) Relationships: is a type of negative regulation of tolerance induction dependent upon immune response [GO:0002653]; is a type of GO:0002655; negatively regulates GO:0002462 Definition: Any process that stops, prevents, or reduces the frequency, rate, or extent of tolerance induction to nonself antigen. Also known as: down regulation of tolerance induction to nonself antigen, down-regulation of tolerance induction to nonself antigen, downregulation of tolerance induction to nonself antigen, inhibition of tolerance induction to nonself antigen Sources: GOC:add